response to stimulus involved in regulation of muscle adaptation [GO:0014874] (BP) Relationships: is a type of response to stimulus [GO:0050896]; is part of GO:0043502 Definition: Any process that results in a change in state or activity of a cell or an organism (in terms of movement, secretion, enzyme production, gene expression, etc.) as a result of a stimulus. This occurs as part of the regulation of muscle adaptation. Sources: GOC:ef, GOC:mtg_muscle Also known as: response to stimulus involved in regulation of muscle plasticity Subtypes: GO:0014873, response to injury involved in regulation of muscle adaptation [GO:0014876], GO:0014877, response to electrical stimulus involved in regulation of muscle adaptation [GO:0014878]